{
  "gene_name": "Serine_threonine-protein kinase H1",
  "gene": "UniProtKB:P11801",
  "term_id": "UNKNOWN:0002",
  "gene_symbol": "PSKH1",
  "term_label": "Unknown biological process"
}